mitochondrial pyruvate dehydrogenase (lipoamide) phosphatase complex [GO:0019910] (CC) Definition: A mitochondrial complex of a regulatory and catalytic subunit that catalyzes the dephosphorylation and concomitant reactivation of the alpha subunit of the E1 component of the pyruvate dehydrogenase complex. An example of this component is found in Mus musculus. References: PMID:9395502 Sources: GOC:mtg_sensu Note: See also the cellular component term 'mitochondrial pyruvate dehydrogenase complex ; GO:0005967'. Relationships: is a type of pyruvate dehydrogenase (lipoamide) phosphatase complex [GO:0045253]; is a type of GO:0098798; is part of mitochondrial matrix [GO:0005759]